acetyl-CoA transmembrane transport [GO:0035348] (biological process) Sources: GO:bf Relationships: is a type of GO:0015876; is a type of purine-containing compound transmembrane transport [GO:0072530] Definition: The process in which acetyl-CoA is transported across a membrane. Acetyl-CoA is a derivative of coenzyme A in which the sulfhydryl group is acetylated; it is a metabolite derived from several pathways (e.g. glycolysis, fatty acid oxidation, amino-acid catabolism) and is further metabolized by the tricarboxylic acid cycle. It is a key intermediate in lipid and terpenoid biosynthesis. Also known as: acetyl-CoA membrane transport Note: Note that this term is not intended for use in annotating lateral movement within membranes.